{
  "gene_name": "Dynein regulatory complex subunit 7",
  "term_label": "flagellated sperm motility",
  "term_id": "GO:0030317",
  "gene_symbol": "DRC7",
  "gene": "UniProtKB:Q8IY82"
}